{
  "term_label": "voltage-gated calcium channel activity",
  "term_id": "GO:0005245",
  "gene_name": "Polycystin-2",
  "gene": "UniProtKB:Q13563",
  "gene_symbol": "PKD2"
}